{
  "gene_name": "G antigen 12J",
  "gene": "UniProtKB:A6NER3",
  "gene_symbol": "GAGE12J",
  "term_id": "UNKNOWN:0002",
  "term_label": "Unknown biological process"
}